{
  "gene": "UniProtKB:Q96PZ2",
  "gene_symbol": "FAM111A",
  "term_label": "serine-type peptidase activity",
  "term_id": "GO:0008236",
  "gene_name": "Serine protease FAM111A"
}